{
  "gene_name": "Zinc finger protein 747",
  "term_label": "nucleus",
  "gene_symbol": "ZNF747",
  "gene": "UniProtKB:Q9BV97",
  "term_id": "GO:0005634"
}